endoplasmic reticulum tubular network maintenance [GO:0071788] (biological process) Definition: The organization process that preserves the endoplasmic reticulum (ER) tubular network in a stable functional or structural state. The ER tubular network is the ER part that comprises the membranes with high curvature in cross-section. Also known as: ER tubular network maintenance Relationships: is a type of cellular component maintenance [GO:0043954]; is a type of endoplasmic reticulum tubular network organization [GO:0071786] References: PMID:16469703, PMID:20434336 Sources: GOC:mah